{
  "gene_name": "Putative nucleosome assembly protein 1-like 6",
  "term_label": "Unknown biological process",
  "gene": "UniProtKB:A6NFF2",
  "term_id": "UNKNOWN:0002",
  "gene_symbol": "NAP1L6P"
}